regulation of alpha-beta T cell activation [GO:0046634] (BP) Also known as: regulation of alpha-beta T lymphocyte activation, regulation of alpha-beta T-cell activation, regulation of alpha-beta T-lymphocyte activation Subtypes: GO:0046635, negative regulation of alpha-beta T cell activation [GO:0046636], regulation of alpha-beta T cell differentiation [GO:0046637], GO:0046640, regulation of NK T cell activation [GO:0051133], regulation of CD4-positive, alpha-beta T cell activation [GO:2000514], regulation of CD8-positive, alpha-beta T cell activation [GO:2001185] Relationships: is a type of regulation of T cell activation [GO:0050863]; regulates alpha-beta T cell activation [GO:0046631] Definition: Any process that modulates the frequency, rate or extent of alpha-beta T cell activation. Sources: GOC:ai